{
  "term_label": "cytoplasm",
  "gene": "UniProtKB:Q6N069",
  "term_id": "GO:0005737",
  "gene_name": "N-alpha-acetyltransferase 16, NatA auxiliary subunit",
  "gene_symbol": "NAA16"
}